homoserine dehydrogenase activity [GO:0004412] (molecular function) Definition: Catalysis of the reaction: L-homoserine + NADP+ = L-aspartate-4-semialdehyde + NADPH + H+. Relationships: is a type of oxidoreductase activity, acting on the CH-OH group of donors, NAD or NADP as acceptor [GO:0016616] Sources: EC:1.1.1.3